pheromone metabolic process [GO:0042810] (biological process) Definition: The chemical reactions and pathways involving pheromones, a substance that is secreted and released by an organism and detected by a second organism of the same or a closely related species, in which it causes a specific reaction, such as a definite behavioral reaction or a developmental process. Sources: ISBN:0198506732 Also known as: pheromone metabolism Relationships: is a type of secondary metabolic process [GO:0019748]; is a type of hormone metabolic process [GO:0042445] Subtypes: GO:0042811, pheromone catabolic process [GO:0042812]